{
  "term_label": "nucleotide-excision repair",
  "term_id": "GO:0006289",
  "gene": "UniProtKB:Q9BX63",
  "gene_name": "Fanconi anemia group J protein",
  "gene_symbol": "BRIP1"
}